embryonic meristem initiation [GO:0090421] (biological process) Definition: Initiation of a region of tissue in a plant embryo that is composed of one or more undifferentiated cells capable of undergoing mitosis and differentiation. Sources: GOC:tb Relationships: is a type of GO:0010014 Subtypes: root meristem specification [GO:0010071], primary shoot apical meristem specification [GO:0010072]